cellular response to L-glutamate [GO:1905232] (biological process) Definition: Any process that results in a change in state or activity of a cell (in terms of movement, secretion, enzyme production, gene expression, etc.) as a result of a L-glutamate(1-) stimulus. References: PMID:25962137 Sources: GOC:TermGenie, GO_REF:0000071 Relationships: is a type of GO:0071230; is a type of cellular response to nitrogen compound [GO:1901699]; is a type of cellular response to oxygen-containing compound [GO:1901701]; is a type of response to L-glutamate [GO:1902065] Also known as: cellular response to L-glutamate(1-)